{
  "gene": "UniProtKB:Q01826",
  "term_label": "chromatin remodeling",
  "gene_name": "DNA-binding protein SATB1",
  "term_id": "GO:0006338",
  "gene_symbol": "SATB1"
}